(R)-limonene 6-monooxygenase activity [GO:0052741] (molecular function) Also known as: (R)-limonene,NADPH:oxygen oxidoreductase (6-hydroxylating) activity, (+)-limonene 6-monooxygenase activity, (+)-limonene-6-hydroxylase activity Definition: Catalysis of the reaction: (4R)-limonene + O2 + reduced [NADPH--hemoprotein reductase] = (1R,5S)-carveol + H+ + H2O + oxidized [NADPH--hemoprotein reductase]. Relationships: is a type of oxidoreductase activity, acting on paired donors, with incorporation or reduction of molecular oxygen, reduced flavin or flavoprotein as one donor, and incorporation of one atom of oxygen [GO:0016712]; is a type of GO:0019113 Sources: RHEA:18957